{
  "gene": "UniProtKB:Q9BXW4",
  "term_id": "GO:0000045",
  "gene_name": "Microtubule-associated proteins 1A_1B light chain 3C",
  "gene_symbol": "MAP1LC3C",
  "term_label": "autophagosome assembly"
}